regulation of tetrapyrrole metabolic process [GO:1901401] (biological process) Definition: Any process that modulates the frequency, rate or extent of tetrapyrrole metabolic process. Subtypes: regulation of chlorophyll metabolic process [GO:0090056], regulation of cobalamin metabolic process [GO:0106064], regulation of tetrapyrrole catabolic process [GO:1901404], regulation of tetrapyrrole biosynthetic process [GO:1901463] Sources: GOC:TermGenie, GOC:mengo_curators Also known as: regulation of tetrapyrrole metabolism Relationships: is_a GO:0019222; regulates tetrapyrrole metabolic process [GO:0033013]